{
  "gene_symbol": "RAC1",
  "term_label": "cytoskeleton",
  "term_id": "GO:0005856",
  "gene_name": "Ras-related C3 botulinum toxin substrate 1",
  "gene": "UniProtKB:P63000"
}